{
  "gene_symbol": "LRPPRC",
  "term_label": "regulation of mitochondrial translation",
  "gene_name": "Leucine-rich PPR motif-containing protein, mitochondrial",
  "term_id": "GO:0070129",
  "gene": "UniProtKB:P42704"
}